xanthine metabolic process [GO:0046110] (biological process) Definition: The chemical reactions and pathways involving xanthine, 2,6-dihydroxypurine, a purine formed in the metabolic breakdown of guanine but not present in nucleic acids. Sources: GOC:go_curators Also known as: xanthine metabolism Relationships: is a type of purine nucleobase metabolic process [GO:0006144] Subtypes: GO:0009115, GO:0046111